{
  "term_label": "endomembrane system",
  "term_id": "GO:0012505",
  "gene": "UniProtKB:Q9UMX5",
  "gene_name": "Neudesin",
  "gene_symbol": "NENF"
}